{
  "term_id": "UNKNOWN:0001",
  "gene_symbol": "RTTN",
  "term_label": "Unknown molecular function",
  "gene_name": "Rotatin",
  "gene": "UniProtKB:Q86VV8"
}